{
  "gene_symbol": "FGF1",
  "gene": "UniProtKB:P05230",
  "gene_name": "Fibroblast growth factor 1",
  "term_id": "GO:0043410",
  "term_label": "positive regulation of MAPK cascade"
}